mannose metabolic process [GO:0006013] (biological process) Sources: ISBN:0198506732 Definition: The chemical reactions and pathways involving mannose, the aldohexose manno-hexose, the C-2 epimer of glucose. The D-(+)-form is widely distributed in mannans and hemicelluloses and is of major importance in the core oligosaccharide of N-linked oligosaccharides of glycoproteins. Subtypes: mannose biosynthetic process [GO:0019307], GO:0019309, GO:0061728 Also known as: mannose metabolism Relationships: is a type of GO:0019318